{
  "gene_symbol": "PLEKHH3",
  "term_id": "UNKNOWN:0001",
  "term_label": "Unknown molecular function",
  "gene_name": "Pleckstrin homology domain-containing family H member 3",
  "gene": "UniProtKB:Q7Z736"
}